UCG codon-amino acid adaptor activity [GO:0033408] (molecular function) Relationships: is a type of triplet codon-amino acid adaptor activity [GO:0030533] Also known as: TCG codon-amino acid adaptor activity, serine tRNA Definition: A triplet codon-amino acid adaptor activity that recognizes a UCG codon. Note: Note that in the standard genetic code, TCG codes for serine. Sources: GOC:mah